{
  "gene": "UniProtKB:Q9BW61",
  "gene_symbol": "DDA1",
  "gene_name": "DET1- and DDB1-associated protein 1",
  "term_id": "GO:0080008",
  "term_label": "Cul4-RING E3 ubiquitin ligase complex"
}